{
  "gene": "UniProtKB:Q96SE7",
  "gene_name": "Zinc finger protein 347",
  "gene_symbol": "ZNF347",
  "term_id": "GO:0006357",
  "term_label": "regulation of transcription by RNA polymerase II"
}